{
  "gene_name": "Cadherin-6",
  "term_label": "adherens junction organization",
  "gene_symbol": "CDH6",
  "gene": "UniProtKB:P55285",
  "term_id": "GO:0034332"
}